{
  "term_label": "polytene chromosome",
  "term_id": "GO:0005700",
  "gene_symbol": "KMT5A",
  "gene_name": "N-lysine methyltransferase KMT5A",
  "gene": "UniProtKB:Q9NQR1"
}